{
  "term_label": "Unknown cellular component",
  "gene": "UniProtKB:Q8NGU2",
  "gene_symbol": "OR9A4",
  "term_id": "UNKNOWN:0003",
  "gene_name": "Olfactory receptor 9A4"
}